{
  "gene_name": "Transmembrane protein 202",
  "term_label": "Unknown molecular function",
  "gene_symbol": "TMEM202",
  "term_id": "UNKNOWN:0001",
  "gene": "UniProtKB:A6NGA9"
}